{
  "term_label": "proteasome-mediated ubiquitin-dependent protein catabolic process",
  "gene_name": "Sharpin",
  "gene": "UniProtKB:Q9H0F6",
  "term_id": "GO:0043161",
  "gene_symbol": "SHARPIN"
}